{
  "term_label": "RNA polymerase II cis-regulatory region sequence-specific DNA binding",
  "term_id": "GO:0000978",
  "gene_name": "Zinc finger protein GLI2",
  "gene": "UniProtKB:P10070",
  "gene_symbol": "GLI2"
}